{
  "term_label": "spindle assembly",
  "gene_name": "Microtubule-associated protein RP_EB family member 1",
  "term_id": "GO:0051225",
  "gene": "UniProtKB:Q15691",
  "gene_symbol": "MAPRE1"
}